negative regulation of protein localization to centrosome [GO:1904780] (biological process) Definition: Any process that stops, prevents or reduces the frequency, rate or extent of protein localization to centrosome. Note: An example is cdk-2 in C. elegans (UniProt ID O61847) in PMID:17115027 (inferred from mutant phenotype). Relationships: is a type of GO:1903828; is a type of regulation of protein localization to centrosome [GO:1904779]; negatively regulates protein localization to centrosome [GO:0071539] References: PMID:17115027 Sources: GOC:TermGenie, GO_REF:0000058 Also known as: down regulation of protein localisation to centrosome, down regulation of protein localization to centrosome, down-regulation of protein localisation to centrosome, down-regulation of protein localization to centrosome, downregulation of protein localisation to centrosome, downregulation of protein localization to centrosome, negative regulation of protein localisation to centrosome, inhibition of protein localisation to centrosome, inhibition of protein localization to centrosome